{
  "term_id": "GO:0007007",
  "gene_name": "Transmembrane protein 11, mitochondrial",
  "gene": "UniProtKB:P17152",
  "gene_symbol": "TMEM11",
  "term_label": "inner mitochondrial membrane organization"
}